{
  "gene_symbol": "NKAIN4",
  "gene_name": "Sodium_potassium-transporting ATPase subunit beta-1-interacting protein 4",
  "term_id": "UNKNOWN:0003",
  "gene": "UniProtKB:Q8IVV8",
  "term_label": "Unknown cellular component"
}